synaptic transmission, cholinergic [GO:0007271] (biological process) Also known as: cholinergic synaptic transmission Regulation: regulated by regulation of synaptic transmission, cholinergic [GO:0032222]; RO_0002212 by negative regulation of synaptic transmission, cholinergic [GO:0032223]; positively regulated by positive regulation of synaptic transmission, cholinergic [GO:0032224] Relationships: is a type of chemical synaptic transmission [GO:0007268] Definition: The vesicular release of acetylcholine from a presynapse, across a chemical synapse, the subsequent activation of dopamine receptors at the postsynapse of a target cell (neuron, muscle, or secretory cell) and the effects of this activation on the postsynaptic membrane potential and ionic composition of the postsynaptic cytosol. This process encompasses both spontaneous and evoked release of neurotransmitter and all parts of synaptic vesicle exocytosis. Evoked transmission starts with the arrival of an action potential at the presynapse. Sources: GOC:dos, Wikipedia:Cholinergic